{
  "gene": "UniProtKB:P62308",
  "term_label": "U2-type prespliceosome",
  "gene_name": "Small nuclear ribonucleoprotein G",
  "gene_symbol": "SNRPG",
  "term_id": "GO:0071004"
}